{
  "term_label": "Unknown biological process",
  "gene": "UniProtKB:A2A2Z9",
  "gene_symbol": "ANKRD18B",
  "gene_name": "Ankyrin repeat domain-containing protein 18B",
  "term_id": "UNKNOWN:0002"
}